{
  "gene": "UniProtKB:Q96MY1",
  "term_id": "UNKNOWN:0003",
  "gene_name": "Nucleolar protein 4-like",
  "gene_symbol": "NOL4L",
  "term_label": "Unknown cellular component"
}